{
  "gene": "UniProtKB:Q13275",
  "term_id": "GO:0071526",
  "gene_symbol": "SEMA3F",
  "term_label": "semaphorin-plexin signaling pathway",
  "gene_name": "Semaphorin-3F"
}